regulation of supramolecular fiber organization [GO:1902903] (biological process) References: PMID:23921388 Sources: GOC:PARL, GOC:TermGenie, GOC:rl, GO_REF:0000058 Note: HSPA8, human, P11142 in PMID:23921388 inferred from direct assay to negatively regulate fibrillation of alpha-Syn in vitro Subtypes: GO:0031113, GO:0031114, GO:0043519, regulation of sarcomere organization [GO:0060297], GO:0110053, GO:1902904, positive regulation of supramolecular fiber organization [GO:1902905], GO:1905304, regulation of amyloid fibril formation [GO:1905906] Relationships: is_a regulation of cellular component organization [GO:0051128]; regulates supramolecular fiber organization [GO:0097435] Also known as: regulation of fibril organisation Definition: Any process that modulates the frequency, rate or extent of supramolecular fiber organization.